{
  "gene_name": "NAD-dependent protein deacylase sirtuin-5, mitochondrial",
  "term_label": "Unknown biological process",
  "gene": "UniProtKB:Q9NXA8",
  "gene_symbol": "SIRT5",
  "term_id": "UNKNOWN:0002"
}